symbiont-mediated activation of host signal transduction pathway via agonism of host cell surface receptor [GO:0141134] (biological process) Definition: A process in which a symbiont subverts a signal transduction pathway in the host organism by binding to and enhancing the activation of the receptor of the pathway. The host is defined as the larger of the organisms involved in a symbiotic interaction. References: PMID:10221874, PMID:18563600 Also known as: symbiont-mediated perturbation of host signal transduction pathway via antagonism of host cell surface receptor Relationships: is a type of symbiont-mediated activation of host signal transduction pathway [GO:0052028]